{
  "gene_name": "Pleckstrin homology domain-containing family B member 2",
  "gene_symbol": "PLEKHB2",
  "term_id": "GO:0045595",
  "gene": "UniProtKB:Q96CS7",
  "term_label": "regulation of cell differentiation"
}